{
  "term_id": "UNKNOWN:0002",
  "term_label": "Unknown biological process",
  "gene_name": "Small ribosomal subunit protein uS10m",
  "gene": "UniProtKB:P82664",
  "gene_symbol": "MRPS10"
}